{
  "term_label": "Unknown molecular function",
  "term_id": "UNKNOWN:0001",
  "gene_name": "NADH dehydrogenase [ubiquinone] 1 alpha subcomplex subunit 2",
  "gene": "UniProtKB:O43678",
  "gene_symbol": "NDUFA2"
}